{
  "gene_symbol": "ZCCHC8",
  "term_id": "GO:0071013",
  "gene_name": "Zinc finger CCHC domain-containing protein 8",
  "gene": "UniProtKB:Q6NZY4",
  "term_label": "catalytic step 2 spliceosome"
}